cytosol to Golgi apparatus transport [GO:0140820] (biological process) Subtypes: GDP-fucose import into Golgi lumen [GO:0036085], UDP-beta-L-arabinofuranose import into Golgi lumen [GO:0140821], GO:1904257 Relationships: is_a transmembrane transport [GO:0055085] References: PMID:28373556 Definition: The directed movement of substances from the cytosol into the Golgi apparatus of a cell.